{
  "gene_symbol": "CENPM",
  "gene_name": "Centromere protein M",
  "term_label": "Unknown molecular function",
  "term_id": "UNKNOWN:0001",
  "gene": "UniProtKB:Q9NSP4"
}